{
  "term_label": "histone H3K4me3 reader activity",
  "gene_symbol": "MORC3",
  "gene": "UniProtKB:Q14149",
  "term_id": "GO:0140002",
  "gene_name": "MORC family CW-type zinc finger protein 3"
}